{
  "term_id": "GO:0005096",
  "gene_name": "TBC1 domain family member 3G",
  "gene": "UniProtKB:Q6DHY5",
  "gene_symbol": "TBC1D3G",
  "term_label": "GTPase activator activity"
}